{
  "gene_symbol": "LILRB5",
  "term_id": "GO:0002767",
  "gene_name": "Leukocyte immunoglobulin-like receptor subfamily B member 5",
  "term_label": "immune response-inhibiting cell surface receptor signaling pathway",
  "gene": "UniProtKB:O75023"
}